positive regulation of interleukin-22 production [GO:0032746] (biological process) Definition: Any process that activates or increases the frequency, rate, or extent of interleukin-22 production. Relationships: is a type of positive regulation of cytokine production [GO:0001819]; is a type of regulation of interleukin-22 production [GO:0032666]; positively regulates interleukin-22 production [GO:0032626] Sources: GOC:mah Also known as: positive regulation of IL-22 production, up regulation of interleukin-22 production, up-regulation of interleukin-22 production, upregulation of interleukin-22 production, activation of interleukin-22 production, positive regulation of interleukin-22 biosynthetic process, stimulation of interleukin-22 production